{
  "term_id": "GO:0035591",
  "gene_symbol": "GAB3",
  "gene": "UniProtKB:Q8WWW8",
  "gene_name": "GRB2-associated-binding protein 3",
  "term_label": "signaling adaptor activity"
}